{
  "gene": "UniProtKB:Q9Y3A6",
  "gene_name": "Transmembrane emp24 domain-containing protein 5",
  "term_id": "GO:0006888",
  "gene_symbol": "TMED5",
  "term_label": "endoplasmic reticulum to Golgi vesicle-mediated transport"
}